{
  "gene_symbol": "PRKCE",
  "gene": "UniProtKB:Q02156",
  "term_id": "GO:0035556",
  "term_label": "intracellular signal transduction",
  "gene_name": "Protein kinase C epsilon type"
}